{
  "term_label": "(3S)-3-hydroxyacyl-CoA dehydrogenase (NAD+) activity",
  "gene": "UniProtKB:Q16836",
  "term_id": "GO:0003857",
  "gene_name": "Hydroxyacyl-coenzyme A dehydrogenase, mitochondrial",
  "gene_symbol": "HADH"
}